{
  "term_id": "GO:0005886",
  "gene_name": "Olfactory receptor 6S1",
  "gene_symbol": "OR6S1",
  "term_label": "plasma membrane",
  "gene": "UniProtKB:Q8NH40"
}